{
  "gene": "UniProtKB:A0A075B714",
  "term_id": "UNKNOWN:0001",
  "gene_symbol": "TRAJ7",
  "gene_name": "T cell receptor alpha joining 7 (Fragment)",
  "term_label": "Unknown molecular function"
}